epithelial cell migration [GO:0010631] (biological process) Relationships: is_a ameboidal-type cell migration [GO:0001667]; is part of GO:0090132 Sources: GOC:BHF, GOC:ascb_2009, GOC:dph, GOC:tb Definition: The orderly movement of an epithelial cell from one site to another, often during the development of a multicellular organism. Subtypes: follicle cell of egg chamber migration [GO:0007297], epithelial cell migration, open tracheal system [GO:0007427], GO:0051546, cell migration involved in prostatic bud elongation [GO:0060518], cell migration involved in mammary placode formation [GO:0060619], corneal epithelial cell migration [GO:0061581], intestinal epithelial cell migration [GO:0061582], GO:0072155, GO:0090521, melanocyte migration [GO:0097324] Regulation: regulated by regulation of epithelial cell migration [GO:0010632]; negatively regulated by negative regulation of epithelial cell migration [GO:0010633]; positively regulated by positive regulation of epithelial cell migration [GO:0010634]